supraspliceosomal complex [GO:0044530] (cellular component) Relationships: is a type of GO:0005681 References: PMID:19282290 Sources: GOC:ans, GOC:jl Definition: Multicomponent complex of RNA and proteins that is composed of four active spliceosomes, termed native spliceosomes, connected to each other by the pre-mRNA. The supraspliceosome is the nuclear machine where the pre-mRNA processing takes place, like the 5'-end capping, 3'-end cleavage, splicing and editing. Also known as: supraspliceosome complex